negative regulation of presynaptic cytosolic calcium concentration [GO:0099113] (BP) Sources: GOC:dos Relationships: is a type of negative regulation of cytosolic calcium ion concentration [GO:0051481]; occurs in presynapse [GO:0098793] Definition: Any process that decreases the concentration of calcium ions in the presynaptic cytosol.